tRNA methyltransferase complex [GO:0043527] (cellular component) References: PMID:24904644, PMID:9851972 Sources: GOC:jl Relationships: is a type of GO:0034708 Subtypes: tRNA (m1A) methyltransferase complex [GO:0031515], tRNA (m2G10) methyltransferase complex [GO:0043528], tRNA (m7G46) methyltransferase complex [GO:0106143] Definition: A multimeric protein complex involved in the methylation of specific nucleotides in tRNA.